{
  "term_label": "positive regulation of TORC1 signaling",
  "gene_name": "WW domain-containing adapter protein with coiled-coil",
  "gene_symbol": "WAC",
  "term_id": "GO:1904263",
  "gene": "UniProtKB:Q9BTA9"
}